regulation of megakaryocyte differentiation [GO:0045652] (BP) Subtypes: negative regulation of megakaryocyte differentiation [GO:0045653], GO:0045654 Definition: Any process that modulates the frequency, rate or extent of megakaryocyte differentiation. Relationships: is a type of GO:0045637; regulates GO:0030219 Sources: GOC:go_curators